phosphatidylinositol-1,4,5-trisphosphate 5-phosphatase activity [GO:0052867] (molecular function) Relationships: is a type of GO:0034594; is a type of phosphatidylinositol phosphate 5-phosphatase activity [GO:0034595] Also known as: PtdIns(1,4,5)P(3) phosphatase activity, PtdIns(1,4,5)P3 phosphatase activity, phosphatidyl-myo-inositol-1,4,5-trisphosphate phosphatase activity, phosphatidylinositol 1,4,5-trisphosphate phosphatase activity, phosphatidylinositol-trisphosphatase activity, triphosphoinositide phosphatase activity, triphosphoinositide phosphomonoesterase activity Sources: GOC:curators Definition: Catalysis of the reaction: phosphatidyl-1D-myo-inositol 1,4,5-trisphosphate + H2O = 1-phosphatidyl-1D-myo-inositol 1,4-bisphosphate + phosphate.